{
  "gene": "UniProtKB:P49407",
  "term_label": "cytoplasmic vesicle",
  "gene_symbol": "ARRB1",
  "term_id": "GO:0031410",
  "gene_name": "Beta-arrestin-1"
}